cerebrospinal fluid secretion [GO:0033326] (biological process) Definition: The regulated release of cerebrospinal fluid (CSF) from the choroid plexus of the lateral, third and fourth ventricles. The cerebrospinal fluid is a clear liquid that located within the ventricles, spinal canal, and subarachnoid spaces. References: PMID:10716451 Sources: GOC:ln Also known as: CSF secretion Relationships: is a type of body fluid secretion [GO:0007589]; is a type of secretion by tissue [GO:0032941]